{
  "gene_symbol": "GABRG1",
  "gene": "UniProtKB:Q8N1C3",
  "gene_name": "Gamma-aminobutyric acid receptor subunit gamma-1",
  "term_id": "GO:0032590",
  "term_label": "dendrite membrane"
}